{
  "gene": "UniProtKB:Q16585",
  "term_label": "Unknown molecular function",
  "term_id": "UNKNOWN:0001",
  "gene_symbol": "SGCB",
  "gene_name": "Beta-sarcoglycan"
}